{
  "gene_name": "SPARC-related modular calcium-binding protein 2",
  "term_id": "GO:0005604",
  "gene_symbol": "SMOC2",
  "gene": "UniProtKB:Q9H3U7",
  "term_label": "basement membrane"
}